deoxyadenosine catabolic process [GO:0006157] (biological process) Also known as: deoxyadenosine breakdown, deoxyadenosine catabolism, deoxyadenosine degradation, deoxyadenosine phosphorolysis Definition: The chemical reactions and pathways resulting in the breakdown of deoxyadenosine, 2-deoxyribosyladenine, one of the four major nucleosides of DNA. Sources: GOC:go_curators Relationships: is a type of deoxyadenosine metabolic process [GO:0046090]; is a type of purine deoxyribonucleoside catabolic process [GO:0046124]